{
  "gene": "UniProtKB:Q99616",
  "term_id": "GO:0048020",
  "gene_name": "C-C motif chemokine 13",
  "gene_symbol": "CCL13",
  "term_label": "CCR chemokine receptor binding"
}